{
  "gene": "UniProtKB:A6NMZ7",
  "term_label": "extracellular matrix organization",
  "gene_symbol": "COL6A6",
  "term_id": "GO:0030198",
  "gene_name": "Collagen alpha-6(VI) chain"
}